{
  "gene_symbol": "ARRDC4",
  "term_id": "GO:0005737",
  "gene": "UniProtKB:Q8NCT1",
  "term_label": "cytoplasm",
  "gene_name": "Arrestin domain-containing protein 4"
}